{
  "gene_name": "Ribitol-5-phosphate transferase FKTN",
  "term_label": "Golgi membrane",
  "gene_symbol": "FKTN",
  "gene": "UniProtKB:O75072",
  "term_id": "GO:0000139"
}